{
  "gene_symbol": "PKD2L1",
  "term_id": "GO:0005262",
  "gene": "UniProtKB:Q9P0L9",
  "term_label": "calcium channel activity",
  "gene_name": "Polycystin-2-like protein 1"
}